{
  "term_id": "GO:0005634",
  "gene_symbol": "MCM2",
  "term_label": "nucleus",
  "gene": "UniProtKB:P49736",
  "gene_name": "DNA replication licensing factor MCM2"
}